thiosulfate transport [GO:0015709] (biological process) Also known as: thiosulphate transport Definition: The directed movement of thiosulfate into, out of or within a cell, or between cells, by means of some agent such as a transporter or pore. Relationships: is_a GO:0015698; is a type of GO:0072348 Sources: GOC:krc